{
  "gene_name": "Hsc70-interacting protein",
  "gene_symbol": "ST13",
  "term_label": "protein folding",
  "term_id": "GO:0006457",
  "gene": "UniProtKB:P50502"
}